ciliary membrane [GO:0060170] (cellular component) Sources: GOC:cilia, GOC:dph, GOC:rph Definition: The portion of the plasma membrane surrounding a cilium. Subtypes: ciliary pocket membrane [GO:0020018], photoreceptor outer segment membrane [GO:0042622], non-motile cilium membrane [GO:0098804], cone photoreceptor disc membrane [GO:0120201] Note: Note that cilia and eukaryotic flagella are deemed to be equivalent. Also known as: cilial membrane, cilium membrane, flagellar membrane, flagellum membrane Relationships: is a type of cell projection membrane [GO:0031253]; is a type of bounding membrane of organelle [GO:0098588]; is part of cilium [GO:0005929]